neural keel formation [GO:0014025] (biological process) Definition: The formation of a thickened region of the neurectoderm that is roughly triangular in cross section. The neural keel develops from the neural plate and develops into the neural rod. Neural keel formation occurs during primary neurulation in teleosts. Sources: GOC:dh, GOC:ef Relationships: is a type of anatomical structure formation involved in morphogenesis [GO:0048646]; is part of GO:0014023